{
  "gene_symbol": "PRPF40A",
  "gene": "UniProtKB:O75400",
  "gene_name": "Pre-mRNA-processing factor 40 homolog A",
  "term_label": "RNA binding",
  "term_id": "GO:0003723"
}